beta-galactoside alpha-2,6-sialyltransferase activity [GO:0003835] (molecular function) Definition: Catalysis of the reaction: CMP-N-acetylneuraminate + beta-D-galactoside = N-acetyl-alpha-neuraminyl-(2->6)-beta-D-galactosyl derivative + CMP + H+. Sources: EC:2.4.3.1 Also known as: beta-galactosamide alpha-2,6-sialyltransferase activity, beta-galactoside alpha-(2,6)-sialyltransferase, CMP-N-acetylneuraminate-beta-galactosamide-alpha-2,6-sialyltransferase activity, lactosylceramide alpha-2,6-N-sialyltransferase Relationships: is a type of sialyltransferase activity [GO:0008373]